{
  "gene_name": "F-box only protein 27",
  "term_id": "GO:0006516",
  "gene_symbol": "FBXO27",
  "term_label": "glycoprotein catabolic process",
  "gene": "UniProtKB:Q8NI29"
}